Wnt signaling pathway involved in forebrain neuroblast division [GO:0021874] (biological process) Also known as: Wnt receptor signaling pathway involved in forebrain neuroblast division, Wnt receptor signalling pathway in forebrain neuroblast division, Wnt-activated signaling pathway involved in forebrain neuroblast division References: PMID:16226447 Sources: GOC:cls, GOC:dgh, GOC:dph, GOC:jid, GO_REF:0000021 Relationships: is a type of Wnt signaling pathway [GO:0016055]; is part of GO:0021873 Definition: The series of molecular signals initiated by binding of Wnt protein to a receptor on the surface of the target cell that contributes to the self renewal of neuroblasts in the forebrain.